{
  "gene_name": "C2 domain-containing protein 5",
  "gene_symbol": "C2CD5",
  "term_id": "GO:0005886",
  "term_label": "plasma membrane",
  "gene": "UniProtKB:Q86YS7"
}